{
  "term_label": "cell fate commitment",
  "gene": "UniProtKB:P04628",
  "term_id": "GO:0045165",
  "gene_symbol": "WNT1",
  "gene_name": "Proto-oncogene Wnt-1"
}